ubiquitin-like ligase-substrate adaptor activity [GO:1990756] (molecular function) References: PMID:24658274 Definition: The binding activity of a molecule that brings together a ubiquitin-like ligase (including ubiquitin ligase and UFM1 ligase) and its substrate. Usually mediated by F-box BTB/POZ domain proteins. Relationships: is a type of enzyme-substrate adaptor activity [GO:0140767] Also known as: protein binding, bridging involved in substrate recognition for ubiquitination, ubiquitin ligase substrate adaptor, UFM1 ligase-substrate adaptor activity, ubiquitin ligase-substrate adaptor activity